synaptic vesicle recycling via endosome [GO:0036466] (biological process) Definition: Synaptic vesicle recycling where vesicles endocytosed via clathrin-coated pits re-acidify and refill with neurotransmitters after passing through an endosomal intermediate. Regulation: regulated by regulation of recycling endosome localization within postsynapse [GO:0099158] References: PMID:15217342 Sources: GOC:PARL, GOC:aruk, GOC:bc, GOC:bf, GOC:dos Also known as: recycling endosome localization within postsynapse Relationships: is a type of synaptic vesicle recycling [GO:0036465]; is a type of intracellular transport [GO:0046907]; is part of synaptic vesicle endosomal processing [GO:0099532]